GPI-anchor transamidase complex [GO:0042765] (cellular component) Definition: An enzyme complex which in humans and yeast consists of at least five proteins; for example, the complex contains GAA1, GPI8, PIG-S, PIG-U, and PIG-T in human, and Gaa1p, Gab1p, Gpi8p, Gpi16p, and Gpi17p in yeast. Catalyzes the posttranslational attachment of the carboxy-terminus of a precursor protein to a GPI-anchor. Relationships: is a type of caspase complex [GO:0008303]; is a type of membrane protein complex [GO:0098796]; is a type of endoplasmic reticulum protein-containing complex [GO:0140534]; is a type of GO:1990234; is part of endoplasmic reticulum membrane [GO:0005789] References: PMID:12802054 Sources: GOC:jl, GOC:rb Also known as: GPIT complex Note: Note that this term should not be confused with 'glycosylphosphatidylinositol-N-acetylglucosaminyltransferase (GPI-GnT) complex ; GO:0000506', which represents a distinct complex with a different catalytic activity.